{
  "term_label": "mitochondrial intermembrane space chaperone complex",
  "gene_symbol": "TIMM10B",
  "gene": "UniProtKB:Q9Y5J6",
  "gene_name": "Mitochondrial import inner membrane translocase subunit Tim10 B",
  "term_id": "GO:0042719"
}